{
  "gene_name": "DNA damage-regulated autophagy modulator protein 2",
  "term_label": "photoreceptor cell maintenance",
  "gene_symbol": "DRAM2",
  "term_id": "GO:0045494",
  "gene": "UniProtKB:Q6UX65"
}